{
  "gene": "UniProtKB:P78333",
  "gene_name": "Glypican-5",
  "term_id": "GO:0090263",
  "term_label": "positive regulation of canonical Wnt signaling pathway",
  "gene_symbol": "GPC5"
}